{
  "term_id": "GO:0003713",
  "gene_symbol": "CITED4",
  "gene": "UniProtKB:Q96RK1",
  "term_label": "transcription coactivator activity",
  "gene_name": "Cbp_p300-interacting transactivator 4"
}